{
  "gene": "UniProtKB:Q9Y261",
  "gene_name": "Hepatocyte nuclear factor 3-beta",
  "gene_symbol": "FOXA2",
  "term_id": "GO:0000981",
  "term_label": "DNA-binding transcription factor activity, RNA polymerase II-specific"
}